{
  "gene_name": "Carbohydrate sulfotransferase 8",
  "term_label": "proteoglycan biosynthetic process",
  "term_id": "GO:0030166",
  "gene_symbol": "CHST8",
  "gene": "UniProtKB:Q9H2A9"
}